acetylgalactosaminyl-O-glycosyl-glycoprotein beta-1,6-N-acetylglucosaminyltransferase activity [GO:0047225] (molecular function) Definition: Catalysis of the reaction: N-acetyl-beta-D-glucosaminyl-1,3-N-acetyl-D-galactosaminyl-R + UDP-N-acetyl-D-glucosamine = N-acetyl-beta-D-glucosaminyl-1,6-(N-acetyl-beta-D-glucosaminyl-1,3)-N-acetyl-D-galactosaminyl-R + UDP. Also known as: O-glycosyl-oligosaccharide-glycoprotein N-acetylglucosaminyltransferase IV activity, UDP-N-acetyl-D-glucosamine:O-oligosaccharide-glycoprotein (N-acetyl-D-glucosamine to N-acetyl-D-galactosamine of N-acetyl-beta-D-glucosaminyl-1,3-N-acetyl-D-galactosaminyl-R) beta-1,6-N-acetyl-D-glucosaminyltransferase activity, core 4 beta6-GalNAc-transferase activity, core 6-beta-GalNAc-transferase B activity, core 6beta-GalNAc-transferase B, uridine diphosphoacetylglucosamine-mucin beta(1->6)-acetylglucosaminyltransferase B Sources: EC:2.4.1.148 Relationships: is a type of acetylglucosaminyltransferase activity [GO:0008375]; is_a GO:0140103